{
  "gene": "UniProtKB:Q96CP7",
  "term_label": "plasma membrane organization",
  "gene_name": "TLC domain-containing protein 1",
  "gene_symbol": "TLCD1",
  "term_id": "GO:0007009"
}